{
  "gene_symbol": "CDC42EP5",
  "term_id": "GO:0031274",
  "gene_name": "Cdc42 effector protein 5",
  "term_label": "positive regulation of pseudopodium assembly",
  "gene": "UniProtKB:Q6NZY7"
}